negative regulation of macrophage inflammatory protein 1 alpha production [GO:0071641] (biological process) Sources: GOC:mah Definition: Any process that stops, prevents, or reduces the frequency, rate, or extent of production of macrophage inflammatory protein 1 alpha. Also known as: negative regulation of macrophage inflammatory protein production, negative regulation of CCL3 production, negative regulation of MIP-1a production, negative regulation of chemokine (C-C motif) ligand 3 production Relationships: is a type of negative regulation of chemokine production [GO:0032682]; is_a regulation of macrophage inflammatory protein 1 alpha production [GO:0071640]; negatively regulates macrophage inflammatory protein-1 alpha production [GO:0071608]